{
  "gene_symbol": "TREM2",
  "term_id": "GO:0004888",
  "gene_name": "Triggering receptor expressed on myeloid cells 2",
  "term_label": "transmembrane signaling receptor activity",
  "gene": "UniProtKB:Q9NZC2"
}